{
  "term_label": "RNA polymerase II cis-regulatory region sequence-specific DNA binding",
  "gene_name": "Zinc finger protein 578",
  "gene": "UniProtKB:Q96N58",
  "term_id": "GO:0000978",
  "gene_symbol": "ZNF578"
}